{
  "term_label": "cellular response to amino acid stimulus",
  "term_id": "GO:0071230",
  "gene_symbol": "LAMTOR2",
  "gene_name": "Ragulator complex protein LAMTOR2",
  "gene": "UniProtKB:Q9Y2Q5"
}